positive regulation of myotube differentiation [GO:0010831] (biological process) Relationships: is a type of GO:0010830; is a type of positive regulation of striated muscle cell differentiation [GO:0051155]; positively regulates myotube differentiation [GO:0014902] Sources: GOC:dph, GOC:tb Definition: Any process that activates, maintains or increases the frequency, rate or extent of myotube differentiation. Myotube differentiation is the process in which a relatively unspecialized cell acquires specialized features of a myotube cell. Myotubes are multinucleated cells that are formed when proliferating myoblasts exit the cell cycle, differentiate and fuse. Subtypes: GO:1902811